GTP synthesis coupled proton transport [GO:0015987] (biological process) Relationships: is a type of energy coupled proton transport, down electrochemical gradient [GO:0015985] Definition: The transport of protons across a membrane to generate an electrochemical gradient (proton-motive force) that powers GTP synthesis. Sources: ISBN:0716731363